{
  "term_id": "GO:0061630",
  "term_label": "ubiquitin protein ligase activity",
  "gene_name": "E3 ubiquitin-protein ligase pellino homolog 1",
  "gene_symbol": "PELI1",
  "gene": "UniProtKB:Q96FA3"
}